{
  "gene": "UniProtKB:Q8IV08",
  "term_label": "Unknown biological process",
  "gene_symbol": "PLD3",
  "term_id": "UNKNOWN:0002",
  "gene_name": "5'-3' exonuclease PLD3"
}